{
  "gene_symbol": "CX3CR1",
  "gene": "UniProtKB:P49238",
  "term_label": "external side of plasma membrane",
  "term_id": "GO:0009897",
  "gene_name": "CX3C chemokine receptor 1"
}